{
  "term_label": "Unknown molecular function",
  "gene_symbol": "NDRG4",
  "gene": "UniProtKB:Q9ULP0",
  "gene_name": "Protein NDRG4",
  "term_id": "UNKNOWN:0001"
}